{
  "gene": "UniProtKB:Q9ULU4",
  "term_id": "UNKNOWN:0002",
  "gene_symbol": "ZMYND8",
  "gene_name": "MYND-type zinc finger-containing chromatin reader ZMYND8",
  "term_label": "Unknown biological process"
}